{
  "term_id": "GO:0005886",
  "gene": "UniProtKB:P35613",
  "gene_symbol": "BSG",
  "gene_name": "Basigin",
  "term_label": "plasma membrane"
}